{
  "gene_symbol": "PHOX2B",
  "gene": "UniProtKB:Q99453",
  "term_id": "GO:0048666",
  "gene_name": "Paired mesoderm homeobox protein 2B",
  "term_label": "neuron development"
}